{
  "gene": "UniProtKB:P48751",
  "gene_name": "Anion exchange protein 3",
  "gene_symbol": "SLC4A3",
  "term_label": "regulation of intracellular pH",
  "term_id": "GO:0051453"
}